{
  "gene_name": "26S proteasome non-ATPase regulatory subunit 8",
  "term_id": "GO:0005634",
  "gene": "UniProtKB:P48556",
  "term_label": "nucleus",
  "gene_symbol": "PSMD8"
}